{
  "term_id": "GO:0016279",
  "term_label": "protein-lysine N-methyltransferase activity",
  "gene_name": "Histone-lysine N-methyltransferase SETD7",
  "gene_symbol": "SETD7",
  "gene": "UniProtKB:Q8WTS6"
}